cellular response to monosaccharide stimulus [GO:0071326] (biological process) Subtypes: GO:0071298, cellular response to hexose stimulus [GO:0071331], cellular response to glyceraldehyde [GO:1905631] Definition: Any process that results in a change in state or activity of a cell (in terms of movement, secretion, enzyme production, gene expression, etc.) as a result of a monosaccharide stimulus. Relationships: is a type of response to monosaccharide [GO:0034284]; is a type of cellular response to carbohydrate stimulus [GO:0071322] Sources: GOC:mah